{
  "term_id": "GO:0004674",
  "gene_symbol": "CSNK1G1",
  "term_label": "protein serine/threonine kinase activity",
  "gene_name": "Casein kinase I isoform gamma-1",
  "gene": "UniProtKB:Q9HCP0"
}